{
  "gene": "UniProtKB:Q9H9B1",
  "gene_name": "Histone-lysine N-methyltransferase EHMT1",
  "term_label": "chromatin",
  "term_id": "GO:0000785",
  "gene_symbol": "EHMT1"
}